{
  "term_label": "double-strand break repair via homologous recombination",
  "gene_name": "Zinc finger SWIM domain-containing protein 7",
  "gene_symbol": "ZSWIM7",
  "gene": "UniProtKB:Q19AV6",
  "term_id": "GO:0000724"
}